{
  "term_id": "GO:0000388",
  "gene_name": "U5 small nuclear ribonucleoprotein 200 kDa helicase",
  "gene": "UniProtKB:O75643",
  "gene_symbol": "SNRNP200",
  "term_label": "spliceosome conformational change to release U4 (or U4atac) and U1 (or U11)"
}